positive regulation of circadian rhythm [GO:0042753] (biological process) Also known as: up regulation of circadian rhythm, up-regulation of circadian rhythm, upregulation of circadian rhythm, activation of circadian rhythm, stimulation of circadian rhythm Sources: GOC:go_curators Definition: Any process that activates or increases the frequency, rate or extent of a circadian rhythm behavior. Subtypes: positive regulation of circadian sleep/wake cycle, wakefulness [GO:0010841], positive regulation of circadian sleep/wake cycle, sleep [GO:0045938], GO:1904061 Relationships: is a type of regulation of circadian rhythm [GO:0042752]; is a type of positive regulation of biological process [GO:0048518]; positively regulates circadian rhythm [GO:0007623]